{
  "gene": "UniProtKB:Q9NZ71",
  "term_label": "telomeric loop disassembly",
  "gene_name": "Regulator of telomere elongation helicase 1",
  "gene_symbol": "RTEL1",
  "term_id": "GO:0090657"
}